{
  "term_label": "synaptic vesicle",
  "term_id": "GO:0008021",
  "gene_symbol": "PICALM",
  "gene_name": "Phosphatidylinositol-binding clathrin assembly protein",
  "gene": "UniProtKB:Q13492"
}